{
  "gene_symbol": "ZFYVE27",
  "gene": "UniProtKB:Q5T4F4",
  "term_label": "positive regulation of axon extension",
  "term_id": "GO:0045773",
  "gene_name": "Protrudin"
}